{
  "term_id": "GO:0042742",
  "gene": "UniProtKB:P05161",
  "gene_name": "Ubiquitin-like protein ISG15",
  "gene_symbol": "ISG15",
  "term_label": "defense response to bacterium"
}